{
  "term_id": "UNKNOWN:0001",
  "term_label": "Unknown molecular function",
  "gene": "UniProtKB:Q7Z7C7",
  "gene_name": "Stimulated by retinoic acid gene 8 protein homolog",
  "gene_symbol": "STRA8"
}